{
  "term_id": "GO:0030036",
  "term_label": "actin cytoskeleton organization",
  "gene": "UniProtKB:Q96KR7",
  "gene_name": "Phosphatase and actin regulator 3",
  "gene_symbol": "PHACTR3"
}